{
  "gene": "UniProtKB:Q01813",
  "term_label": "fructose 1,6-bisphosphate metabolic process",
  "gene_symbol": "PFKP",
  "term_id": "GO:0030388",
  "gene_name": "ATP-dependent 6-phosphofructokinase, platelet type"
}